{
  "gene": "UniProtKB:Q6UWZ7",
  "term_id": "GO:0008017",
  "gene_symbol": "ABRAXAS1",
  "term_label": "microtubule binding",
  "gene_name": "BRCA1-A complex subunit Abraxas 1"
}